regulation of immunological synapse formation [GO:2000520] (biological process) Subtypes: negative regulation of immunological synapse formation [GO:2000521], GO:2000522 Relationships: is a type of regulation of lymphocyte activation [GO:0051249]; regulates immunological synapse formation [GO:0001771] Also known as: regulation of formation of immunological synapse Sources: GOC:obol Definition: Any process that modulates the frequency, rate or extent of immunological synapse formation.